2,4,5-trichlorophenoxyacetic acid catabolic process [GO:0046228] (biological process) Relationships: is a type of benzene-containing compound metabolic process [GO:0042537]; is a type of monocarboxylic acid catabolic process [GO:0072329]; is a type of organohalogen metabolic process [GO:0090345]; is a type of ether catabolic process [GO:1901502] Sources: GOC:ai Definition: The chemical reactions and pathways resulting in the breakdown of 2,4,5-trichlorophenoxyacetic acid, a chlorinated aromatic compound widely used as a herbicide. Also known as: 2,4,5-trichlorophenoxyacetic acid breakdown, 2,4,5-trichlorophenoxyacetic acid catabolism, 2,4,5-trichlorophenoxyacetic acid degradation